{
  "term_label": "Unknown cellular component",
  "gene_symbol": "IGHV1-24",
  "term_id": "UNKNOWN:0003",
  "gene": "UniProtKB:A0A0C4DH33",
  "gene_name": "Immunoglobulin heavy variable 1-24"
}